{
  "gene_symbol": "RINL",
  "term_id": "GO:0005829",
  "term_label": "cytosol",
  "gene": "UniProtKB:Q6ZS11",
  "gene_name": "Ras and Rab interactor-like protein"
}